5-carboxymethyl-2-hydroxymuconic-semialdehyde dehydrogenase activity [GO:0018480] (molecular function) Also known as: 5-carboxymethyl-2-hydroxymuconic-semialdehyde:NAD+ oxidoreductase activity, carboxymethylhydroxymuconic semialdehyde dehydrogenase activity Definition: Catalysis of the reaction: 5-carboxymethyl-2-hydroxymuconate semialdehyde + H2O + NAD+ = 5-carboxymethyl-2-hydroxymuconate + NADH + H+. Sources: EC:1.2.1.60 Relationships: is a type of oxidoreductase activity, acting on the aldehyde or oxo group of donors, NAD or NADP as acceptor [GO:0016620]